apyrase activity [GO:0004050] (molecular function) Definition: Catalysis of the reaction: a ribonucleoside 5'-triphosphate + 2 H2O = a ribonucleoside 5'-phosphate + 2 phosphate. This reaction consists of two distinct successive phosphate-releasing steps, with NDPs as intermediates. Apyrases are active against both di- and triphosphate nucleotides (NDPs and NTPs) and hydrolyze NTPs to nucleotide monophosphates (NMPs). Relationships: is a type of pyrophosphatase activity [GO:0016462] Sources: EC:3.6.1.5